glucuronoxylan 4-O-methyltransferase activity [GO:0030775] (molecular function) Definition: Catalysis of the reaction: S-adenosyl-L-methionine + glucuronoxylan D-glucuronate = S-adenosyl-L-homocysteine + glucuronoxylan 4-O-methyl-D-glucuronate. Sources: EC:2.1.1.112 Relationships: is a type of GO:0008757 Also known as: S-adenosyl-L-methionine:glucuronoxylan-D-glucuronate 4-O-methyltransferase activity